isoleucyl-tRNA aminoacylation [GO:0006428] (BP) Definition: The process of coupling isoleucine to isoleucyl-tRNA, catalyzed by isoleucyl-tRNA synthetase. The isoleucyl-tRNA synthetase is a class-I synthetase. The activated amino acid is transferred to the 2'-OH group of a isoleucine-accetping tRNA. The 2'-O-aminoacyl-tRNA will ultimately migrate to the 3' position via transesterification. Sources: GOC:mcc, ISBN:0716730510 Relationships: is_a tRNA aminoacylation for protein translation [GO:0006418] Subtypes: GO:0070152